intestinal epithelial cell differentiation [GO:0060575] (biological process) Relationships: is a type of columnar/cuboidal epithelial cell differentiation [GO:0002065]; is part of digestive tract development [GO:0048565] Sources: GOC:dph Definition: The process in which a relatively unspecialized cell acquires specialized features of a columnar/cuboidal epithelial cell of the intestine. Subtypes: interstitial cell of Cajal differentiation [GO:0061453], GO:1903703